detection of injury involved in regulation of muscle adaptation [GO:0014885] (biological process) Definition: The series of events by which an injury stimulus is received and converted into a molecular signal. This occurs as part of the regulation of muscle adaptation. Sources: GOC:ef, GOC:mtg_muscle Relationships: is a type of detection of wounding [GO:0014822]; is a type of response to injury involved in regulation of muscle adaptation [GO:0014876] Also known as: detection of injury involved in regulation of muscle plasticity